response to manganese-induced endoplasmic reticulum stress [GO:1990737] (BP) Definition: Any process that results in a change in state or activity of a cell (in terms of movement, secretion, enzyme production, gene expression, etc.) as a result of endoplasmic reticulum stress caused by a manganese stimulus. Also known as: manganese-induced ER stress response, response to Mn-induced ER stress, response to manganese-induced ER stress References: PMID:23934647 Sources: GOC:PARL, GOC:bf Relationships: is a type of response to endoplasmic reticulum stress [GO:0034976]; is a type of cellular response to chemical stress [GO:0062197]; is a type of cellular response to manganese ion [GO:0071287]